{
  "term_id": "GO:0005634",
  "gene_name": "Homeobox protein Nkx-3.1",
  "gene": "UniProtKB:Q99801",
  "gene_symbol": "NKX3-1",
  "term_label": "nucleus"
}